histone acetyltransferase regulator activity [GO:0035034] (molecular function) Note: See also the molecular function term 'histone acetyltransferase activity ; GO:0004402'. Relationships: is a type of enzyme regulator activity [GO:0030234]; has part histone acetyltransferase binding [GO:0035035]; regulates histone acetyltransferase activity [GO:0004402] Also known as: histone acetylase regulator activity Sources: GOC:bf Definition: Binds to and modulates the activity of histone acetyltransferase.